regulation of blood pressure [GO:0008217] (biological process) Also known as: blood pressure regulation, blood pressure homeostasis, control of blood pressure Relationships: is a type of GO:0065008; BFO_0000050 GO:0008015 Definition: Any process that modulates the force with which blood travels through the circulatory system. The process is controlled by a balance of processes that increase pressure and decrease pressure. Sources: GOC:dph, GOC:mtg_cardio, ISBN:0721643949 Subtypes: regulation of systemic arterial blood pressure [GO:0003073], regulation of blood pressure by chemoreceptor signaling pathway [GO:0010850], GO:0014916, negative regulation of blood pressure [GO:0045776], positive regulation of blood pressure [GO:0045777]